positive regulation of nematode male tail tip morphogenesis [GO:0110039] (biological process) Definition: Any process that activates or increases the frequency, rate or extent of nematode male tail tip morphogenesis. References: PMID:28068334 Sources: GOC:rz Relationships: is a type of positive regulation of developmental process [GO:0051094]; is a type of positive regulation of multicellular organismal process [GO:0051240]; is a type of GO:0110037; positively regulates nematode male tail tip morphogenesis [GO:0045138]